{
  "gene_symbol": "LRRC4B",
  "gene": "UniProtKB:Q9NT99",
  "gene_name": "Leucine-rich repeat-containing protein 4B",
  "term_id": "GO:0099560",
  "term_label": "synaptic membrane adhesion"
}